{
  "gene_name": "Cytosolic 10-formyltetrahydrofolate dehydrogenase",
  "gene": "UniProtKB:O75891",
  "term_id": "GO:0016155",
  "gene_symbol": "ALDH1L1",
  "term_label": "formyltetrahydrofolate dehydrogenase activity"
}